{
  "gene_symbol": "TMEM105",
  "term_label": "Unknown molecular function",
  "term_id": "UNKNOWN:0001",
  "gene_name": "Transmembrane protein 105",
  "gene": "UniProtKB:Q8N8V8"
}